{
  "gene_name": "Putative olfactory receptor 2I1",
  "term_label": "olfactory receptor activity",
  "term_id": "GO:0004984",
  "gene": "UniProtKB:Q8NGU4",
  "gene_symbol": "OR2I1"
}